{
  "term_id": "UNKNOWN:0002",
  "gene_name": "Putative protein ATXN8OS",
  "gene": "UniProtKB:P0DMR3",
  "term_label": "Unknown biological process",
  "gene_symbol": "ATXN8OS"
}